{
  "gene_symbol": "LCE3B",
  "term_label": "Unknown molecular function",
  "gene": "UniProtKB:Q5TA77",
  "gene_name": "Late cornified envelope protein 3B",
  "term_id": "UNKNOWN:0001"
}